{
  "gene_symbol": "HPGDS",
  "gene": "UniProtKB:O60760",
  "gene_name": "Hematopoietic prostaglandin D synthase",
  "term_id": "GO:0004364",
  "term_label": "glutathione transferase activity"
}